{
  "term_label": "detection of chemical stimulus involved in sensory perception of smell",
  "gene_name": "Olfactory receptor 2B6",
  "gene": "UniProtKB:P58173",
  "term_id": "GO:0050911",
  "gene_symbol": "OR2B6"
}